{
  "gene_name": "Beta-sarcoglycan",
  "term_id": "GO:0016012",
  "gene_symbol": "SGCB",
  "term_label": "sarcoglycan complex",
  "gene": "UniProtKB:Q16585"
}